positive regulation of tetrapyrrole biosynthetic process [GO:1901465] (biological process) Subtypes: GO:0070455, positive regulation of tetrapyrrole biosynthetic process from glutamate [GO:1901412], GO:1901415, positive regulation of chlorophyll biosynthetic process [GO:1902326] Relationships: is a type of positive regulation of biosynthetic process [GO:0009891]; is a type of regulation of tetrapyrrole biosynthetic process [GO:1901463]; positively regulates tetrapyrrole biosynthetic process [GO:0033014] Definition: Any process that activates or increases the frequency, rate or extent of tetrapyrrole biosynthetic process. Also known as: activation of tetrapyrrole anabolism, activation of tetrapyrrole biosynthesis, activation of tetrapyrrole formation, activation of tetrapyrrole synthesis, positive regulation of tetrapyrrole anabolism, positive regulation of tetrapyrrole biosynthesis, positive regulation of tetrapyrrole formation, positive regulation of tetrapyrrole synthesis, up regulation of tetrapyrrole anabolism, up regulation of tetrapyrrole biosynthesis, up regulation of tetrapyrrole biosynthetic process, up regulation of tetrapyrrole formation, up regulation of tetrapyrrole synthesis, up-regulation of tetrapyrrole anabolism, up-regulation of tetrapyrrole biosynthesis, up-regulation of tetrapyrrole biosynthetic process, up-regulation of tetrapyrrole formation, up-regulation of tetrapyrrole synthesis, upregulation of tetrapyrrole anabolism, upregulation of tetrapyrrole biosynthesis, upregulation of tetrapyrrole biosynthetic process, upregulation of tetrapyrrole formation, upregulation of tetrapyrrole synthesis, activation of tetrapyrrole biosynthetic process Sources: GOC:TermGenie, GOC:mengo_curators